thelarche [GO:0042695] (biological process) Definition: The beginning of development of the breasts in the female. References: PMID:19117864 Sources: GOC:curators Relationships: is a type of GO:0046543; BFO_0000050 mammary gland development [GO:0030879]